{
  "gene_symbol": "PCDHA3",
  "term_id": "GO:0005886",
  "gene_name": "Protocadherin alpha-3",
  "gene": "UniProtKB:Q9Y5H8",
  "term_label": "plasma membrane"
}